apical dendrite morphogenesis [GO:0150021] (BP) Definition: The process in which the anatomical structures of an apical dendrite are generated and organized. Relationships: is a type of dendrite morphogenesis [GO:0048813]; is part of apical dendrite development [GO:0150022] Subtypes: apical dendrite arborization [GO:0150023] References: PMID:22683681 Sources: GOC:aruk, GOC:bc